{
  "term_label": "ubiquitin-like protein ligase binding",
  "gene": "UniProtKB:Q6EEV6",
  "gene_symbol": "SUMO4",
  "term_id": "GO:0044389",
  "gene_name": "Small ubiquitin-related modifier 4"
}